gas vesicle organization [GO:0031412] (biological process) Also known as: gas vesicle organisation, gas vesicle biosynthesis, gas vesicle formation, gas vesicle organization and biogenesis Definition: A process that is carried out at the cellular level which results in the assembly, arrangement of constituent parts, or disassembly of a gas vesicle. A gas vesicle is a hollow structure made of protein, which usually has the form of a cylindrical tube closed by conical end caps. Note: Note that although gas vesicles are commonly referred to as 'vesicles' or 'vacuoles' in the literature, they are not surrounded by a membrane. Relationships: is_a organelle organization [GO:0006996] Sources: GOC:mah